{
  "gene": "UniProtKB:P41235",
  "term_id": "GO:0004879",
  "gene_name": "Hepatocyte nuclear factor 4-alpha",
  "gene_symbol": "HNF4A",
  "term_label": "nuclear receptor activity"
}